{
  "gene_symbol": "MLN",
  "gene": "UniProtKB:P12872",
  "term_id": "GO:0031788",
  "gene_name": "Promotilin",
  "term_label": "motilin receptor binding"
}